tyrosine-ester sulfotransferase activity [GO:0017067] (molecular function) Definition: Catalysis of the reaction: 3'-phospho-5'-adenylyl sulfate + L-tyrosine methyl ester = L-tyrosine methyl ester 4-sulfate + adenosine 3',5'-diphosphate + H+. Also known as: tyrosine-ester sulphotransferase activity, 3'-phosphoadenylyl-sulfate:L-tyrosine-methyl-ester sulfotransferase activity, L-tyrosine methyl ester sulfotransferase activity, aryl sulfotransferase IV Sources: EC:2.8.2.9, RHEA:19977 Relationships: is a type of sulfotransferase activity [GO:0008146]